{
  "term_label": "Unknown cellular component",
  "gene": "UniProtKB:Q9H7Z3",
  "gene_symbol": "NRDE2",
  "term_id": "UNKNOWN:0003",
  "gene_name": "Nuclear exosome regulator NRDE2"
}